{
  "gene": "UniProtKB:P0DW11",
  "term_label": "RNA polymerase II general transcription initiation factor activity",
  "gene_name": "TATA-box-binding protein-associated factor 11-like protein 6",
  "gene_symbol": "TAF11L6",
  "term_id": "GO:0016251"
}